cell aggregation [GO:0098743] (biological process) Definition: The clustering together and adhesion of initially separate cells to form an aggregate. Examples include the clustering of unicellular organisms or blood cells in suspension and the condensation of mesenchymal cells during cartilage formation. Relationships: is a type of cellular process [GO:0009987] Sources: GOC:dos Subtypes: cartilage condensation [GO:0001502], GO:0098630